{
  "term_label": "plasma membrane",
  "gene_symbol": "TRBV9",
  "term_id": "GO:0005886",
  "gene_name": "T cell receptor beta variable 9",
  "gene": "UniProtKB:A0A0B4J1U6"
}